poly-gamma-glutamate biosynthetic process [GO:0070501] (biological process) Definition: The chemical reactions and pathways resulting in the formation of poly-gamma-glutamate, a polymer of D- and/or L-glutamic acid residues linked by gamma-peptidyl bonds. Subtypes: GO:0070502 References: PMID:16689787 Sources: GOC:mah Relationships: is a type of macromolecule biosynthetic process [GO:0009059] Also known as: poly-gamma-glutamate anabolism, poly-gamma-glutamate biosynthesis, poly-gamma-glutamate formation, poly-gamma-glutamate synthesis